{
  "gene_name": "Cytosolic phospholipase A2 beta",
  "term_id": "GO:0005509",
  "term_label": "calcium ion binding",
  "gene_symbol": "PLA2G4B",
  "gene": "UniProtKB:P0C869"
}